{
  "gene_name": "RAD9, HUS1, RAD1-interacting nuclear orphan protein 1",
  "term_label": "DNA damage checkpoint signaling",
  "term_id": "GO:0000077",
  "gene": "UniProtKB:Q9BSD3",
  "gene_symbol": "RHNO1"
}